organelle fusion [GO:0048284] (BP) Subtypes: karyogamy [GO:0000741], mitochondrial fusion [GO:0008053], synaptic vesicle to endosome fusion [GO:0016189], organelle membrane fusion [GO:0090174], GO:0097576, lipid droplet fusion [GO:0160077] Definition: The creation of a single organelle from two or more organelles. Relationships: is a type of organelle organization [GO:0006996] Sources: GOC:jid